{
  "term_id": "GO:0031821",
  "gene_symbol": "GNAI1",
  "gene": "UniProtKB:P63096",
  "gene_name": "Guanine nucleotide-binding protein G(i) subunit alpha-1",
  "term_label": "G protein-coupled serotonin receptor binding"
}